{
  "gene": "UniProtKB:Q8N271",
  "gene_symbol": "PROM2",
  "term_id": "GO:0005902",
  "term_label": "microvillus",
  "gene_name": "Prominin-2"
}